{
  "gene": "UniProtKB:Q9BZW4",
  "gene_symbol": "TM6SF2",
  "gene_name": "Transmembrane 6 superfamily member 2",
  "term_id": "UNKNOWN:0001",
  "term_label": "Unknown molecular function"
}